{
  "gene_name": "E3 SUMO-protein ligase NSE2",
  "gene_symbol": "NSMCE2",
  "gene": "UniProtKB:Q96MF7",
  "term_label": "Smc5-Smc6 complex",
  "term_id": "GO:0030915"
}